{
  "gene": "UniProtKB:Q96PY5",
  "term_label": "cytosol",
  "term_id": "GO:0005829",
  "gene_symbol": "FMNL2",
  "gene_name": "Formin-like protein 2"
}